hypoxia-inducible factor-proline dioxygenase activity [GO:0160082] (molecular function) Also known as: HIF hydroxylase, HIF prolyl hydroxylase Relationships: is a type of peptidyl-proline 4-dioxygenase activity [GO:0031545] Definition: Catalysis of the reaction: 2-oxoglutarate + L-prolyl-[hypoxia-inducible factor alpha subunit] + O2 = CO2 + succinate + trans-4-hydroxy-L-prolyl-[hypoxia-inducible factor alpha subunit]. References: PMID:11595184, PMID:11598268